{
  "term_id": "UNKNOWN:0002",
  "gene_symbol": "PCMTD1",
  "term_label": "Unknown biological process",
  "gene_name": "Protein-L-isoaspartate O-methyltransferase domain-containing protein 1",
  "gene": "UniProtKB:Q96MG8"
}